{
  "gene_name": "R-spondin-2",
  "term_id": "GO:0060173",
  "term_label": "limb development",
  "gene_symbol": "RSPO2",
  "gene": "UniProtKB:Q6UXX9"
}